detection of renal blood flow [GO:0002000] (biological process) Relationships: is a type of detection of mechanical stimulus [GO:0050982]; is part of GO:0001999 Sources: ISBN:0721643949 Definition: The process in which the juxtaglomerular cells of the kidneys receive information about the amount of blood flowing through the arterioles and converts the information to a molecular signal.